{
  "gene": "UniProtKB:Q9BXJ9",
  "gene_symbol": "NAA15",
  "term_label": "Unknown biological process",
  "gene_name": "N-alpha-acetyltransferase 15, NatA auxiliary subunit",
  "term_id": "UNKNOWN:0002"
}